{
  "gene_symbol": "CDH7",
  "gene": "UniProtKB:Q9ULB5",
  "term_id": "GO:0005912",
  "gene_name": "Cadherin-7",
  "term_label": "adherens junction"
}